{
  "gene_symbol": "MTRNR2L11",
  "gene": "UniProtKB:S4R3Y5",
  "term_id": "UNKNOWN:0003",
  "gene_name": "Humanin-like 11",
  "term_label": "Unknown cellular component"
}